{
  "gene_symbol": "PRR30",
  "gene_name": "Proline-rich protein 30",
  "term_id": "UNKNOWN:0002",
  "term_label": "Unknown biological process",
  "gene": "UniProtKB:Q53SZ7"
}